{
  "gene_symbol": "GFI1B",
  "term_id": "GO:0006357",
  "term_label": "regulation of transcription by RNA polymerase II",
  "gene": "UniProtKB:Q5VTD9",
  "gene_name": "Zinc finger protein Gfi-1b"
}